{
  "gene": "UniProtKB:P28325",
  "gene_symbol": "CST5",
  "term_label": "cytoplasm",
  "gene_name": "Cystatin-D",
  "term_id": "GO:0005737"
}